nucleoside transport [GO:0015858] (biological process) Definition: The directed movement of a nucleoside, a nucleobase linked to either beta-D-ribofuranose (ribonucleoside) or 2-deoxy-beta-D-ribofuranose, (a deoxyribonucleotide), into, out of or within a cell, or between cells, by means of some agent such as a transporter or pore. Regulation: regulated by GO:0032242; negatively regulated by GO:0032243; positively regulated by positive regulation of nucleoside transport [GO:0032244] Sources: GOC:ai Relationships: is a type of nucleobase-containing compound transport [GO:0015931]; is_a carbohydrate derivative transport [GO:1901264] Subtypes: intracellular nucleoside transport [GO:0015859], xanthosine transport [GO:0015863], pyrimidine nucleoside transport [GO:0015864], adenosine transport [GO:0032238], nicotinamide riboside transport [GO:0034258], inosine transport [GO:0035340], GO:1901642